anhydrotetracycline monooxygenase activity [GO:0047670] (molecular function) Definition: Catalysis of the reaction: anhydrotetracycline + H+ + NADPH + O2 = 12-dehydrotetracycline + H2O + NADP+. Also known as: ATC oxygenase activity, anhydrotetracycline oxygenase activity, anhydrotetracycline,NADPH:oxygen oxidoreductase (6-hydroxylating) Relationships: is a type of oxidoreductase activity, acting on paired donors, with incorporation or reduction of molecular oxygen, NAD(P)H as one donor, and incorporation of one atom of oxygen [GO:0016709] Sources: EC:1.14.13.38, RHEA:11976